positive regulation of leukocyte migration [GO:0002687] (biological process) Subtypes: GO:0002690, positive regulation of cellular extravasation [GO:0002693], positive regulation of mononuclear cell migration [GO:0071677], GO:1902624, positive regulation of eosinophil migration [GO:2000418] Sources: GOC:add Definition: Any process that activates or increases the frequency, rate, or extent of leukocyte migration. Relationships: is a type of positive regulation of immune system process [GO:0002684]; is a type of GO:0002685; is a type of positive regulation of cell migration [GO:0030335]; positively regulates leukocyte migration [GO:0050900] Also known as: positive regulation of immune cell migration, positive regulation of leucocyte migration, up regulation of leukocyte migration, up-regulation of leukocyte migration, upregulation of leukocyte migration, activation of leukocyte migration, stimulation of leukocyte migration